{
  "term_label": "membrane",
  "gene_symbol": "TSPO",
  "gene_name": "Translocator protein",
  "gene": "UniProtKB:P30536",
  "term_id": "GO:0016020"
}